negative regulation of cell fate commitment [GO:0010454] (biological process) Sources: GOC:dph, GOC:tb Relationships: is a type of regulation of cell fate commitment [GO:0010453]; is_a negative regulation of cell differentiation [GO:0045596]; negatively regulates cell fate commitment [GO:0045165] Subtypes: negative regulation of cell fate specification [GO:0009996], negative regulation of anterior neural cell fate commitment of the neural plate [GO:0022001], negative regulation of sevenless signaling pathway [GO:0045873], GO:0060226, negative regulation of R7 cell fate commitment [GO:0106398], negative regulation of cell fate determination [GO:1905934], negative regulation of establishment or maintenance of neuroblast polarity [GO:2000248], negative regulation of T-helper 17 cell lineage commitment [GO:2000329], negative regulation of venous endothelial cell fate commitment [GO:2000788] Definition: Any process that stops, prevents or reduces the frequency or rate of cell fate commitment. Cell fate commitment is the commitment of cells to specific cell fates and their capacity to differentiate into particular kinds of cells. Positional information is established through protein signals that emanate from a localized source within a cell (the initial one-cell zygote) or within a developmental field.